{
  "term_id": "GO:1901222",
  "gene": "UniProtKB:P50749",
  "gene_name": "Ras association domain-containing protein 2",
  "gene_symbol": "RASSF2",
  "term_label": "regulation of non-canonical NF-kappaB signal transduction"
}